{
  "gene_name": "Ubiquitin-like-conjugating enzyme ATG3",
  "term_label": "Atg8-family conjugating enzyme activity",
  "gene": "UniProtKB:Q9NT62",
  "term_id": "GO:0141046",
  "gene_symbol": "ATG3"
}